{
  "gene_symbol": "NR1H4",
  "gene_name": "Bile acid receptor",
  "term_id": "GO:0030522",
  "gene": "UniProtKB:Q96RI1",
  "term_label": "intracellular receptor signaling pathway"
}